{
  "gene": "UniProtKB:P33993",
  "term_label": "nucleus",
  "gene_name": "DNA replication licensing factor MCM7",
  "term_id": "GO:0005634",
  "gene_symbol": "MCM7"
}